RNA polymerase II C-terminal domain phosphoserine binding [GO:1990269] (molecular function) Definition: Binding to phosphorylated serine residues in the C-terminal domain of RNA polymerase II. References: PMID:22796944 Sources: GOC:di Also known as: RNA Pol II C-terminal domain phosphoserine binding, RNAP II C-terminal domain phosphoserine binding Relationships: is a type of phosphoserine residue binding [GO:0050815]; is a type of GO:0099122